ammeline aminohydrolase activity [GO:0018756] (molecular function) Relationships: is a type of GO:0016813 References: PMID:1991731 Definition: Catalysis of the reaction: ammeline + H2O = ammelide + NH3.